{
  "gene_name": "Olfactory receptor 51M1",
  "term_label": "Unknown biological process",
  "gene_symbol": "OR51M1",
  "term_id": "UNKNOWN:0002",
  "gene": "UniProtKB:Q9H341"
}